{
  "term_label": "ganglioside GM1 binding",
  "gene": "UniProtKB:Q9BZR6",
  "term_id": "GO:1905573",
  "gene_name": "Reticulon-4 receptor",
  "gene_symbol": "RTN4R"
}